vesicle fusion with peroxisome [GO:0019817] (biological process) Definition: The joining of the lipid bilayer membrane around a vesicle with the lipid bilayer membrane around the peroxisome. Sources: GOC:jid Relationships: is_a GO:0006906; is a type of peroxisome organization [GO:0007031]; is part of GO:0007031